{
  "gene_name": "G-protein coupled receptor 12",
  "gene_symbol": "GPR12",
  "gene": "UniProtKB:P47775",
  "term_label": "cytoplasm",
  "term_id": "GO:0005737"
}